{
  "gene_name": "Cation-independent mannose-6-phosphate receptor",
  "term_label": "insulin-like growth factor binding",
  "gene_symbol": "IGF2R",
  "term_id": "GO:0005520",
  "gene": "UniProtKB:P11717"
}